flower formation [GO:0048460] (biological process) Relationships: is a type of developmental process involved in reproduction [GO:0003006]; is a type of anatomical structure formation involved in morphogenesis [GO:0048646]; is part of flower morphogenesis [GO:0048439] Sources: GOC:jid Definition: The process that gives rise to the flower. This process pertains to the initial formation of a structure from unspecified parts.